{
  "gene_symbol": "ADRB2",
  "term_label": "norepinephrine-epinephrine-mediated vasodilation involved in regulation of systemic arterial blood pressure",
  "term_id": "GO:0002025",
  "gene_name": "Beta-2 adrenergic receptor",
  "gene": "UniProtKB:P07550"
}